{
  "term_id": "UNKNOWN:0001",
  "term_label": "Unknown molecular function",
  "gene_symbol": "CFAP53",
  "gene": "UniProtKB:Q96M91",
  "gene_name": "Cilia- and flagella-associated protein 53"
}